{
  "gene": "UniProtKB:Q9NWC5",
  "gene_symbol": "TMEM45A",
  "term_label": "Unknown biological process",
  "gene_name": "Transmembrane protein 45A",
  "term_id": "UNKNOWN:0002"
}